{
  "gene": "UniProtKB:Q13621",
  "term_id": "GO:0008511",
  "term_label": "sodium:potassium:chloride symporter activity",
  "gene_name": "Solute carrier family 12 member 1",
  "gene_symbol": "SLC12A1"
}